{
  "term_id": "GO:0003009",
  "gene_symbol": "TNNI3",
  "gene": "UniProtKB:P19429",
  "term_label": "skeletal muscle contraction",
  "gene_name": "Troponin I, cardiac muscle"
}